{
  "gene_symbol": "HIF3A",
  "term_label": "intracellular oxygen homeostasis",
  "gene": "UniProtKB:Q9Y2N7",
  "gene_name": "Hypoxia-inducible factor 3-alpha",
  "term_id": "GO:0032364"
}